{
  "term_label": "interleukin-2 binding",
  "gene_symbol": "IL2RB",
  "gene_name": "Interleukin-2 receptor subunit beta",
  "term_id": "GO:0019976",
  "gene": "UniProtKB:P14784"
}